posterior commissure morphogenesis [GO:0021961] (biological process) Sources: GOC:cls, GOC:dgh, GOC:dph, GOC:jid, GO_REF:0000021 Definition: Generation of a long process of a CNS neuron, that carries efferent (outgoing) action potentials from the cell body in the midbrain towards target cells in the diencephalon. Relationships: is a type of central nervous system projection neuron axonogenesis [GO:0021952]